gibberellin transmembrane transporter activity [GO:1905201] (molecular function) References: PMID:27139299 Sources: GOC:TermGenie, GO_REF:0000070 Relationships: is a type of carboxylic acid transmembrane transporter activity [GO:0046943]; is a type of lipid transmembrane transporter activity [GO:0170055] Definition: Enables the transfer of gibberellin from one side of a membrane to the other.